{
  "gene": "UniProtKB:Q6X784",
  "gene_symbol": "ZPBP2",
  "term_label": "binding of sperm to zona pellucida",
  "term_id": "GO:0007339",
  "gene_name": "Zona pellucida-binding protein 2"
}